{
  "gene_symbol": "ZNF668",
  "gene": "UniProtKB:Q96K58",
  "term_label": "regulation of transcription by RNA polymerase II",
  "gene_name": "Zinc finger protein 668",
  "term_id": "GO:0006357"
}